6-alpha-maltosylglucose biosynthetic process [GO:0051680] (biological process) Sources: GOC:ai Definition: The chemical reactions and pathways resulting in the formation of 6-alpha-maltosylglucose, also known as isopanose. Also known as: isopanose biosynthesis, isopanose biosynthetic process Relationships: is a type of oligosaccharide biosynthetic process [GO:0009312]